positive regulation of translational elongation [GO:0045901] (biological process) Also known as: up regulation of translational elongation, up-regulation of translational elongation, upregulation of translational elongation, activation of translational elongation, stimulation of translational elongation Sources: GOC:go_curators Subtypes: GO:1900249, positive regulation of selenocysteine incorporation [GO:1904571], GO:1905084, GO:2001126 Relationships: is a type of regulation of translational elongation [GO:0006448]; is a type of GO:0045727; positively regulates translational elongation [GO:0006414] Definition: Any process that activates or increases the frequency, rate or extent of translational elongation.